response to lead ion [GO:0010288] (biological process) Subtypes: cellular response to lead ion [GO:0071284] References: PMID:16461380 Sources: GOC:tair_curators Definition: Any process that results in a change in state or activity of a cell or an organism (in terms of movement, secretion, enzyme production, gene expression, etc.) as a result of a lead ion stimulus. Relationships: is_a GO:0010038